{
  "gene_name": "Protein phosphatase 1J",
  "term_id": "GO:0004741",
  "gene_symbol": "PPM1J",
  "term_label": "[pyruvate dehydrogenase (acetyl-transferring)]-phosphatase activity",
  "gene": "UniProtKB:Q5JR12"
}